{
  "gene": "UniProtKB:Q9UBW5",
  "gene_symbol": "BIN2",
  "term_label": "plasma membrane",
  "term_id": "GO:0005886",
  "gene_name": "Bridging integrator 2"
}